{
  "term_label": "regulation of transcription by RNA polymerase II",
  "term_id": "GO:0006357",
  "gene_name": "Max dimerization protein 4",
  "gene_symbol": "MXD4",
  "gene": "UniProtKB:Q14582"
}